cellular response to amitrole [GO:0072723] (BP) Also known as: cellular response to 3-amino-1,2,4-triazole Relationships: is a type of response to amitrole [GO:0072722]; is a type of GO:1901699 Definition: Any process that results in a change in state or activity of a cell (in terms of movement, secretion, enzyme production, gene expression, etc.) as a result of an amitrole stimulus. Sources: GOC:mah